{
  "gene": "UniProtKB:P16109",
  "gene_symbol": "SELP",
  "term_label": "oligosaccharide binding",
  "term_id": "GO:0070492",
  "gene_name": "P-selectin"
}